cyclic-GMP-AMP hydrolase activity [GO:0106177] (molecular function) Relationships: is a type of hydrolase activity, acting on acid anhydrides, in phosphorus-containing anhydrides [GO:0016818] References: PMID:25344812 Sources: GOC:sp, RHEA:58808 Definition: Catalysis of the reaction: cyclic GMP-AMP + 2 H2O = AMP + GMP.